{
  "term_label": "cytoplasm",
  "gene_symbol": "SH2D6",
  "gene_name": "SH2 domain-containing protein 6",
  "gene": "UniProtKB:Q7Z4S9",
  "term_id": "GO:0005737"
}